{
  "term_id": "GO:0000978",
  "gene": "UniProtKB:Q96EK4",
  "term_label": "RNA polymerase II cis-regulatory region sequence-specific DNA binding",
  "gene_name": "THAP domain-containing protein 11",
  "gene_symbol": "THAP11"
}